{
  "gene_name": "NXPE family member 2",
  "gene": "UniProtKB:Q96DL1",
  "term_id": "UNKNOWN:0001",
  "gene_symbol": "NXPE2",
  "term_label": "Unknown molecular function"
}